prostaglandin J receptor activity [GO:0001785] (molecular function) Definition: Combining with prostaglandin J (PGJ(2)), a metabolite of prostaglandin D (PGD(2)) to initiate a change in cell activity. References: PMID:12878180 Also known as: PGJ(2) receptor activity, PGJ receptor activity Relationships: is a type of prostaglandin receptor activity [GO:0004955]